ventricular trabecula myocardium morphogenesis [GO:0003222] (biological process) Relationships: is a type of ventricular cardiac muscle tissue morphogenesis [GO:0055010]; is a type of heart trabecula morphogenesis [GO:0061384] Sources: GOC:mtg_heart Definition: The process in which the anatomical structures of the trabecular cardiac ventricle muscle are generated and organized. Subtypes: left ventricular trabecular myocardium morphogenesis [GO:0003225], GO:0003227 Also known as: trabecula carnea morphogenesis